{
  "gene_name": "Proton-coupled zinc antiporter SLC30A8",
  "gene_symbol": "SLC30A8",
  "term_label": "insulin secretion",
  "term_id": "GO:0030073",
  "gene": "UniProtKB:Q8IWU4"
}